negative regulation of muscle adaptation [GO:0014745] (biological process) Definition: Any process that stops, prevents, or reduces the frequency, rate, or extent of muscle adaptation. Sources: GOC:mtg_muscle Also known as: negative regulation of muscle plasticity Relationships: is a type of regulation of muscle adaptation [GO:0043502]; is a type of negative regulation of response to stimulus [GO:0048585]; is a type of negative regulation of multicellular organismal process [GO:0051241]; negatively regulates GO:0043500 Subtypes: GO:0010616, negative regulation of muscle atrophy [GO:0014736], negative regulation of muscle hyperplasia [GO:0014740], negative regulation of skeletal muscle hypertrophy [GO:1904205], negative regulation of smooth muscle hypertrophy [GO:1905148]